{
  "gene_name": "Corticosteroid-binding globulin",
  "gene": "UniProtKB:P08185",
  "gene_symbol": "SERPINA6",
  "term_label": "serine-type endopeptidase inhibitor activity",
  "term_id": "GO:0004867"
}